{
  "gene": "UniProtKB:Q8NGE7",
  "gene_symbol": "OR9K2",
  "term_label": "Unknown cellular component",
  "term_id": "UNKNOWN:0003",
  "gene_name": "Olfactory receptor 9K2"
}